{
  "gene_symbol": "SPATA20",
  "term_id": "UNKNOWN:0001",
  "gene": "UniProtKB:Q8TB22",
  "term_label": "Unknown molecular function",
  "gene_name": "Spermatogenesis-associated protein 20"
}